{
  "term_id": "GO:0005737",
  "gene_symbol": "FUBP3",
  "gene_name": "Far upstream element-binding protein 3",
  "gene": "UniProtKB:Q96I24",
  "term_label": "cytoplasm"
}